{
  "gene_symbol": "EIF2AK4",
  "term_label": "eukaryotic translation initiation factor 2alpha kinase activity",
  "term_id": "GO:0004694",
  "gene_name": "eIF-2-alpha kinase GCN2",
  "gene": "UniProtKB:Q9P2K8"
}